{
  "term_id": "GO:0031514",
  "gene_name": "Meiosis-specific nuclear structural protein 1",
  "gene_symbol": "MNS1",
  "term_label": "motile cilium",
  "gene": "UniProtKB:Q8NEH6"
}